neuroblast division in dorsal lateral ganglionic eminence [GO:0021851] (biological process) References: PMID:12626695 Sources: GOC:cls, GOC:dgh, GOC:dph, GOC:jid, GO_REF:0000021 Relationships: is a type of GO:0021848 Definition: The division of neuroblasts in the dorsal region of the lateral ganglionic eminence. These cells give rise to embryonic interneuron precursors that will migrate tangentially to the olfactory bulb.